{
  "term_label": "Unknown cellular component",
  "gene_name": "Probable ATP-dependent RNA helicase DHX34",
  "term_id": "UNKNOWN:0003",
  "gene": "UniProtKB:Q14147",
  "gene_symbol": "DHX34"
}